negative regulation of asexual sporulation resulting in formation of a cellular spore [GO:0043944] (biological process) Relationships: is a type of negative regulation of sporulation resulting in formation of a cellular spore [GO:0042174]; is a type of regulation of asexual sporulation resulting in formation of a cellular spore [GO:0043943]; is a type of negative regulation of asexual reproduction [GO:1903665]; negatively regulates asexual sporulation resulting in formation of a cellular spore [GO:0043936] Definition: Any process that stops, prevents, or reduces the frequency, rate or extent of the formation of a cellular spore derived from the products of mitosis. Subtypes: negative regulation of aeciospore formation [GO:0075250], negative regulation of uredospore formation [GO:0075254], negative regulation of teliospore formation [GO:0075258], negative regulation of sporangiospore formation [GO:0075288] Sources: GOC:pamgo_curators